{
  "term_label": "nucleus",
  "gene": "UniProtKB:Q8IYW5",
  "gene_name": "E3 ubiquitin-protein ligase RNF168",
  "term_id": "GO:0005634",
  "gene_symbol": "RNF168"
}